{
  "gene_symbol": "CYP4F3",
  "term_id": "UNKNOWN:0003",
  "gene_name": "Cytochrome P450 4F3",
  "gene": "UniProtKB:Q08477",
  "term_label": "Unknown cellular component"
}